{
  "gene_name": "Double-stranded RNA-specific editase 1",
  "term_id": "GO:0005737",
  "gene_symbol": "ADARB1",
  "gene": "UniProtKB:P78563",
  "term_label": "cytoplasm"
}